{
  "term_label": "neuropeptide signaling pathway",
  "gene_symbol": "OPRM1",
  "gene_name": "Mu-type opioid receptor",
  "gene": "UniProtKB:P35372",
  "term_id": "GO:0007218"
}